{
  "gene_symbol": "H2AC20",
  "term_id": "GO:0005634",
  "gene_name": "Histone H2A type 2-C",
  "gene": "UniProtKB:Q16777",
  "term_label": "nucleus"
}